{
  "gene": "UniProtKB:Q9Y6X6",
  "gene_name": "Unconventional myosin-XVI",
  "gene_symbol": "MYO16",
  "term_id": "GO:0048471",
  "term_label": "perinuclear region of cytoplasm"
}